cell-cell adhesion involved in synapse maturation [GO:0090125] (biological process) Relationships: is a type of cell-cell adhesion [GO:0098609]; is part of synapse maturation [GO:0060074] Also known as: trans-synaptic adhesion Sources: GOC:ascb_2009, GOC:dph, GOC:tb Definition: The attachment of the pre-synaptic cell to the post-synaptic cell via adhesion molecules that contributes to synapse maturation.